{
  "term_id": "GO:0035861",
  "term_label": "site of double-strand break",
  "gene": "UniProtKB:Q13156",
  "gene_symbol": "RPA4",
  "gene_name": "Replication protein A 30 kDa subunit"
}